{
  "term_id": "UNKNOWN:0001",
  "gene_symbol": "FUNDC1",
  "gene_name": "FUN14 domain-containing protein 1",
  "term_label": "Unknown molecular function",
  "gene": "UniProtKB:Q8IVP5"
}